{
  "gene": "UniProtKB:Q02779",
  "term_id": "GO:0004706",
  "term_label": "JUN kinase kinase kinase activity",
  "gene_symbol": "MAP3K10",
  "gene_name": "Mitogen-activated protein kinase kinase kinase 10"
}